{
  "gene_name": "Forkhead box protein D4",
  "term_label": "DNA-binding transcription factor activity, RNA polymerase II-specific",
  "gene_symbol": "FOXD4",
  "gene": "UniProtKB:Q12950",
  "term_id": "GO:0000981"
}